{
  "term_label": "heme binding",
  "gene_name": "Cytochrome P450 2C8",
  "gene_symbol": "CYP2C8",
  "term_id": "GO:0020037",
  "gene": "UniProtKB:P10632"
}